{
  "term_id": "UNKNOWN:0002",
  "term_label": "Unknown biological process",
  "gene": "UniProtKB:Q9H3U5",
  "gene_name": "Major facilitator superfamily domain-containing protein 1",
  "gene_symbol": "MFSD1"
}